gamma-secretase complex [GO:0070765] (cellular component) Also known as: presenilin complex, CD147-gamma-secretase complex (APH-1a, PS-1, PEN-2, NCT variant), PS1 complex, PS2 complex, gamma-secretase complex (APH1A, PSEN1, PSENEN, NCSTN variant), gamma-secretase complex (APH1A, PSEN2, PSENEN, NCSTN), gamma-secretase complex (APH1B, PSEN1, PSENEN, NCSTN), gamma-secretase complex (APH1B, PSEN2, PSENEN, NCSTN) References: PMID:15286082, PMID:15890777, PMID:17047368, PMID:22122073, PMID:25565961, PMID:28320827, PMID:32616437 Sources: GOC:krc Definition: A protein complex that has aspartic-type endopeptidase activity and contains a presenilin catalytic subunit (either PSEN1 or PSEN2), an APH1 subunit (multiple genes and splice variants exist), nicastrin (NCT), and presenilin enhancer (aka PEN-2 or Psenen), as the core complex. Variants of the complex with different subunit compositions differ in localization and specific substrates. Additionally, variants of the complex exist that contain a additional regulatory subunit as well as the four core subunits; known regulatory subunits include gamma-secretase-activating protein (aka gSAP), TMP1 (aka TMED10), and CD147 antigen (aka basigin). Gamma-secretase cleaves type I transmembrane protein substrates, including the cell surface receptor Notch and the amyloid-beta precursor protein. Relationships: is a type of plasma membrane protein complex [GO:0098797]; is a type of catalytic complex [GO:1902494]